{
  "term_id": "UNKNOWN:0002",
  "gene": "UniProtKB:Q5T870",
  "gene_symbol": "PRR9",
  "gene_name": "Proline-rich protein 9",
  "term_label": "Unknown biological process"
}